aminergic neurotransmitter loading into synaptic vesicle [GO:0015842] (biological process) Sources: GOC:ai Definition: The active transport of aminergic neurotransmitters into a synaptic vesicle. This import is fuelled by an electrochemical gradient across the vesicle membrane, established by the action proton pumps. Relationships: is a type of amine transport [GO:0015837]; is a type of neurotransmitter loading into synaptic vesicle [GO:0098700]